negative regulation of activated T cell proliferation [GO:0046007] (biological process) Relationships: is a type of negative regulation of T cell proliferation [GO:0042130]; is a type of regulation of activated T cell proliferation [GO:0046006]; negatively regulates activated T cell proliferation [GO:0050798] Also known as: down regulation of activated T cell proliferation, down-regulation of activated T cell proliferation, downregulation of activated T cell proliferation, negative regulation of activated T lymphocyte proliferation, negative regulation of activated T-cell proliferation, negative regulation of activated T-lymphocyte proliferation, inhibition of activated T cell proliferation Sources: GOC:go_curators Definition: Any process that stops, prevents or reduces the rate or extent of activated T cell proliferation.